{
  "gene_name": "Receptor-type tyrosine-protein phosphatase U",
  "gene": "UniProtKB:Q92729",
  "term_id": "GO:0004725",
  "gene_symbol": "PTPRU",
  "term_label": "protein tyrosine phosphatase activity"
}